{
  "term_label": "GTPase activator activity",
  "gene_symbol": "EVI5",
  "gene_name": "Ecotropic viral integration site 5 protein homolog",
  "gene": "UniProtKB:O60447",
  "term_id": "GO:0005096"
}